{
  "gene": "UniProtKB:A4FU69",
  "gene_name": "EF-hand calcium-binding domain-containing protein 5",
  "gene_symbol": "EFCAB5",
  "term_id": "UNKNOWN:0002",
  "term_label": "Unknown biological process"
}